carnitine racemase activity [GO:0008809] (MF) Definition: Catalysis of the reaction: D-carnitine = L-carnitine. Sources: MetaCyc:CARNRACE-RXN Relationships: is a type of racemase and epimerase activity, acting on hydroxy acids and derivatives [GO:0016856]